{
  "term_label": "inflammatory response",
  "gene": "UniProtKB:P25090",
  "term_id": "GO:0006954",
  "gene_name": "N-formyl peptide receptor 2",
  "gene_symbol": "FPR2"
}